{
  "term_label": "apical plasma membrane urothelial plaque",
  "gene_name": "Uroplakin-1b",
  "gene_symbol": "UPK1B",
  "gene": "UniProtKB:O75841",
  "term_id": "GO:0120001"
}